{
  "gene": "UniProtKB:P52735",
  "gene_name": "Guanine nucleotide exchange factor VAV2",
  "gene_symbol": "VAV2",
  "term_label": "immune response-regulating cell surface receptor signaling pathway",
  "term_id": "GO:0002768"
}